sporopollenin biosynthetic process [GO:0080110] (biological process) Relationships: is a type of biosynthetic process [GO:0009058]; is part of GO:0010584 References: PMID:19218397 Also known as: sporopollenin biosynthesis Definition: The chemical reactions and pathways resulting in the formation of sporopollenin, a primary constituent of the pollen exine layer.